positive regulation of necroptotic process [GO:0060545] (biological process) Also known as: positive regulation of necroptosis Sources: GOC:BHF, GOC:dph, GOC:mtg_apoptosis, GOC:tb Relationships: is a type of GO:0060544; is a type of GO:0062100; positively regulates GO:0070266 Definition: Any process that increases the rate, frequency or extent of a necroptotic process, a necrotic cell death process that results from the activation of endogenous cellular processes, such as signaling involving death domain receptors or Toll-like receptors.